{
  "gene": "UniProtKB:Q6IQ19",
  "term_id": "GO:1901673",
  "term_label": "regulation of mitotic spindle assembly",
  "gene_symbol": "CCSAP",
  "gene_name": "Centriole, cilia and spindle-associated protein"
}